positive regulation of mechanosensory behavior [GO:1905792] (biological process) Relationships: is_a GO:0032103; is a type of GO:0048520; is a type of regulation of mechanosensory behavior [GO:1905790]; positively regulates mechanosensory behavior [GO:0007638] Definition: Any process that activates or increases the frequency, rate or extent of mechanosensory behavior. Also known as: positive regulation of behavioral response to mechanical stimulus, positive regulation of behavioural response to mechanical stimulus, positive regulation of mechanosensory behaviour, up regulation of behavioral response to mechanical stimulus, up regulation of behavioural response to mechanical stimulus, up regulation of mechanosensory behavior, up regulation of mechanosensory behaviour, up-regulation of behavioral response to mechanical stimulus, up-regulation of behavioural response to mechanical stimulus, up-regulation of mechanosensory behavior, up-regulation of mechanosensory behaviour, upregulation of behavioral response to mechanical stimulus, upregulation of behavioural response to mechanical stimulus, upregulation of mechanosensory behavior, upregulation of mechanosensory behaviour, activation of behavioral response to mechanical stimulus, activation of behavioural response to mechanical stimulus, activation of mechanosensory behavior, activation of mechanosensory behaviour References: PMID:8692859 Sources: GOC:TermGenie, GO_REF:0000058